3-aminopropanal dehydrogenase (NAD+) activity [GO:0102244] (molecular function) Relationships: is a type of aldehyde dehydrogenase (NAD+) activity [GO:0004029] Definition: Catalysis of the reaction: 3-aminopropanal + H2O + NAD+ = beta-alanine + 2 H+ + NADH. Sources: RHEA:30695